proteasome-activating nucleotidase complex [GO:0022623] (cellular component) Also known as: PAN Relationships: is a type of protein-containing complex [GO:0032991]; is part of proteasome accessory complex [GO:0022624] References: PMID:19363223, PMID:19481528 Sources: GOC:bf, GOC:mtg_sensu Definition: A homohexameric complex that recognizes and unfolds core proteasome substrate proteins, and translocates them to the core complex in an ATP dependent manner.